{
  "gene": "UniProtKB:Q8N184",
  "term_id": "GO:0003700",
  "gene_symbol": "ZNF567",
  "term_label": "DNA-binding transcription factor activity",
  "gene_name": "Zinc finger protein 567"
}